{
  "gene_name": "Limbic system-associated membrane protein",
  "gene": "UniProtKB:Q13449",
  "gene_symbol": "LSAMP",
  "term_label": "Unknown molecular function",
  "term_id": "UNKNOWN:0001"
}